{
  "gene_name": "Bardet-Biedl syndrome 2 protein",
  "term_label": "motile cilium",
  "gene_symbol": "BBS2",
  "gene": "UniProtKB:Q9BXC9",
  "term_id": "GO:0031514"
}